{
  "gene": "UniProtKB:Q4V321",
  "term_label": "Unknown molecular function",
  "gene_symbol": "GAGE13",
  "term_id": "UNKNOWN:0001",
  "gene_name": "G antigen 13"
}